{
  "term_id": "GO:0005886",
  "gene_symbol": "OR2T7",
  "gene_name": "Olfactory receptor 2T7",
  "term_label": "plasma membrane",
  "gene": "UniProtKB:P0C7T2"
}